negative regulation of shoot apical meristem development [GO:1902184] (biological process) Also known as: down regulation of promeristem development, down-regulation of promeristem development, downregulation of promeristem development, inhibition of promeristem development, negative regulation of promeristem development, down regulation of SAM development, down regulation of shoot apical meristem development, down-regulation of SAM development, down-regulation of shoot apical meristem development, downregulation of SAM development, downregulation of shoot apical meristem development, inhibition of SAM development, negative regulation of SAM development, inhibition of shoot apical meristem development, down regulation of primary shoot meristem development, down-regulation of primary shoot meristem development, downregulation of primary shoot meristem development, inhibition of primary shoot meristem development, negative regulation of primary shoot meristem development Relationships: is a type of negative regulation of developmental process [GO:0051093]; is a type of regulation of shoot apical meristem development [GO:1902183]; negatively regulates shoot apical meristem development [GO:1902182] References: PMID:21496644 Sources: GOC:TermGenie Definition: Any process that stops, prevents or reduces the frequency, rate or extent of shoot apical meristem development.